{
  "gene_symbol": "MED12L",
  "gene_name": "Mediator of RNA polymerase II transcription subunit 12-like protein",
  "gene": "UniProtKB:Q86YW9",
  "term_label": "mediator complex",
  "term_id": "GO:0016592"
}